{
  "gene_symbol": "CADPS2",
  "gene": "UniProtKB:Q86UW7",
  "gene_name": "Calcium-dependent secretion activator 2",
  "term_label": "glutamatergic synapse",
  "term_id": "GO:0098978"
}